glucose-6-phosphate 3-dehydrogenase activity [GO:0103074] (MF) Definition: Catalysis of the reaction: NAD + D-glucopyranose 6-phosphate = NADH + H+ + 3-dehydro-D-glucose 6-phosphate. Sources: GOC:pz, RHEA:37547 Relationships: is a type of oxidoreductase activity, acting on the CH-OH group of donors, NAD or NADP as acceptor [GO:0016616]